{
  "gene_name": "Large ribosomal subunit protein uL2",
  "gene_symbol": "RPL8",
  "term_id": "GO:0003723",
  "gene": "UniProtKB:P62917",
  "term_label": "RNA binding"
}